{
  "term_label": "cytoskeleton",
  "gene_name": "Keratin, type I cuticular Ha2",
  "gene_symbol": "KRT32",
  "term_id": "GO:0005856",
  "gene": "UniProtKB:Q14532"
}